{
  "gene_symbol": "HNRNPA2B1",
  "gene": "UniProtKB:P22626",
  "gene_name": "Heterogeneous nuclear ribonucleoproteins A2_B1",
  "term_label": "single-stranded telomeric DNA binding",
  "term_id": "GO:0043047"
}